{
  "gene": "UniProtKB:P0DTW3",
  "gene_name": "Probable non-functional immunoglobulin heavy variable 1-38-4",
  "gene_symbol": "IGHV1-38-4",
  "term_id": "UNKNOWN:0003",
  "term_label": "Unknown cellular component"
}